negative regulation of methane biosynthetic process from dimethylamine [GO:1900319] (biological process) Definition: Any process that stops, prevents or reduces the frequency, rate or extent of methane biosynthetic process from dimethylamine. Sources: GOC:TermGenie, GOC:mengo_curators Also known as: down regulation of methane biosynthetic process from dimethylamine, down-regulation of methane biosynthetic process from dimethylamine, downregulation of methane biosynthetic process from dimethylamine, inhibition of methane biosynthetic process from dimethylamine Relationships: is a type of GO:0033239; is a type of regulation of methane biosynthetic process from dimethylamine [GO:1900318]; is a type of negative regulation of alkane biosynthetic process [GO:1901578]; is a type of negative regulation of cellular respiration [GO:1901856]; negatively regulates methane biosynthetic process from dimethylamine [GO:2001129]